bud outgrowth involved in lung branching [GO:0060447] (biological process) Sources: GOC:dph, GOC:mtg_lung Relationships: is a type of branch elongation of an epithelium [GO:0060602]; is part of epithelial tube branching involved in lung morphogenesis [GO:0060441] Regulation: negatively regulated by negative regulation of bud outgrowth involved in lung branching [GO:0061112] Also known as: bud formation involved in lung branching Definition: The process in which a region of the lung epithelium initiates an outgrowth.